{
  "gene_name": "Cylicin-1",
  "gene_symbol": "CYLC1",
  "term_id": "GO:0043159",
  "term_label": "acrosomal matrix",
  "gene": "UniProtKB:P35663"
}